DNA repair complex [GO:1990391] (cellular component) Relationships: is a type of GO:1902494 Also known as: DNA damage repair complex, WHY1 complex Subtypes: GO:0009380, nonhomologous end joining complex [GO:0070419], GO:1990710 Definition: A protein complex involved in DNA repair processes including direct reversal, base excision repair, nucleotide excision repair, photoreactivation, bypass, double-strand break repair pathway, and mismatch repair pathway. References: PMID:17217467, PMID:20551348, PMID:22749910, PMID:24192350 Sources: GOC:bhm